{
  "gene_name": "Protein Wnt-9b",
  "term_id": "GO:0005125",
  "gene_symbol": "WNT9B",
  "gene": "UniProtKB:O14905",
  "term_label": "cytokine activity"
}